bicyclic nitroimidazole catabolic process [GO:0052800] (biological process) Relationships: is a type of nitroimidazole catabolic process [GO:0052804] Subtypes: coenzyme F420-dependent bicyclic nitroimidazole catabolic process [GO:0052799] Also known as: bicyclic nitroimidazole breakdown, bicyclic nitroimidazole catabolism, bicyclic nitroimidazole degradation References: PMID:16387854, PMID:19039139 Definition: The chemical reactions and pathways resulting in the breakdown of a bicyclic nitroimidazole.